{
  "gene": "UniProtKB:Q4VCS5",
  "term_label": "establishment of cell polarity involved in ameboidal cell migration",
  "term_id": "GO:0003365",
  "gene_symbol": "AMOT",
  "gene_name": "Angiomotin"
}